{
  "gene": "UniProtKB:Q9Y267",
  "gene_symbol": "SLC22A14",
  "term_id": "UNKNOWN:0003",
  "term_label": "Unknown cellular component",
  "gene_name": "Solute carrier family 22 member 14"
}